{
  "gene": "UniProtKB:Q14565",
  "gene_symbol": "DMC1",
  "term_id": "GO:0000794",
  "term_label": "condensed nuclear chromosome",
  "gene_name": "Meiotic recombination protein DMC1_LIM15 homolog"
}